{
  "gene": "UniProtKB:Q9UNZ2",
  "gene_symbol": "NSFL1C",
  "term_label": "Golgi organization",
  "gene_name": "NSFL1 cofactor p47",
  "term_id": "GO:0007030"
}